{
  "term_id": "GO:0061709",
  "gene_name": "Autophagy-related protein 9B",
  "gene_symbol": "ATG9B",
  "term_label": "reticulophagy",
  "gene": "UniProtKB:Q674R7"
}